{
  "gene": "UniProtKB:Q2M3R5",
  "term_id": "GO:0051480",
  "term_label": "regulation of cytosolic calcium ion concentration",
  "gene_name": "Solute carrier family 35 member G1",
  "gene_symbol": "SLC35G1"
}